{
  "term_id": "GO:0005634",
  "gene_symbol": "CDK19",
  "term_label": "nucleus",
  "gene_name": "Cyclin-dependent kinase 19",
  "gene": "UniProtKB:Q9BWU1"
}